{
  "term_id": "GO:0005737",
  "gene": "UniProtKB:Q5VT98",
  "gene_symbol": "PRAMEF20",
  "term_label": "cytoplasm",
  "gene_name": "PRAME family member 20"
}